{
  "term_id": "UNKNOWN:0003",
  "gene_name": "Zinc finger protein 285",
  "gene_symbol": "ZNF285",
  "gene": "UniProtKB:Q96NJ3",
  "term_label": "Unknown cellular component"
}